{
  "term_label": "myoblast fusion",
  "gene": "UniProtKB:A0A1B0GTQ4",
  "gene_symbol": "MYMX",
  "term_id": "GO:0007520",
  "gene_name": "Protein myomixer"
}